{
  "term_label": "cell surface",
  "gene": "UniProtKB:O94985",
  "term_id": "GO:0009986",
  "gene_name": "Calsyntenin-1",
  "gene_symbol": "CLSTN1"
}